{
  "term_id": "GO:0004715",
  "term_label": "non-membrane spanning protein tyrosine kinase activity",
  "gene_symbol": "TXK",
  "gene": "UniProtKB:P42681",
  "gene_name": "Tyrosine-protein kinase TXK"
}